{
  "term_id": "UNKNOWN:0003",
  "term_label": "Unknown cellular component",
  "gene": "UniProtKB:O95398",
  "gene_symbol": "RAPGEF3",
  "gene_name": "Rap guanine nucleotide exchange factor 3"
}